{
  "gene_symbol": "IGLV3-12",
  "gene_name": "Immunoglobulin lambda variable 3-12",
  "term_id": "UNKNOWN:0001",
  "term_label": "Unknown molecular function",
  "gene": "UniProtKB:A0A075B6K2"
}